{
  "gene_symbol": "NUCB2",
  "gene_name": "Nucleobindin-2",
  "term_id": "GO:0005509",
  "gene": "UniProtKB:P80303",
  "term_label": "calcium ion binding"
}